{
  "gene_symbol": "CDC40",
  "gene": "UniProtKB:O60508",
  "term_label": "mRNA binding",
  "gene_name": "Pre-mRNA-processing factor 17",
  "term_id": "GO:0003729"
}